opsin binding [GO:0002046] (molecular function) Definition: Binding to an opsin, any of a group of hydrophobic, integral membrane glycoproteins located primarily in the disc membrane of rods or cones, involved in photoreception. Relationships: is a type of protein binding [GO:0005515] Sources: GOC:hjd Also known as: metarhodopsin binding